{
  "term_id": "GO:0035869",
  "gene_symbol": "NPHP4",
  "term_label": "ciliary transition zone",
  "gene_name": "Nephrocystin-4",
  "gene": "UniProtKB:O75161"
}